sulfurtransferase activity [GO:0016783] (molecular function) Also known as: sulphurtransferase activity Sources: EC:2.8.1.-, GOC:ai Relationships: is_a transferase activity, transferring sulphur-containing groups [GO:0016782] Definition: Catalysis of the transfer of sulfur atoms from one compound (donor) to another (acceptor). Subtypes: biotin synthase activity [GO:0004076], GO:0004792, molybdenum cofactor sulfurtransferase activity [GO:0008265], 3-mercaptopyruvate sulfurtransferase activity [GO:0016784], lipoate synthase activity [GO:0016992], molybdopterin synthase activity [GO:0030366], cysteine desulfurase activity [GO:0031071], thiosulfate-dithiol sulfurtransferase activity [GO:0047362], thiosulfate-thiol sulfurtransferase activity [GO:0050337], molybdopterin-synthase sulfurtransferase activity [GO:0061604], tRNA-5-taurinomethyluridine 2-sulfurtransferase [GO:0061708], tRNA-uridine 2-sulfurtransferase activity [GO:0103016], thiosulfate-thioredoxin sulfurtransferase activity [GO:0103041], tRNA-uracil-4 sulfurtransferase activity [GO:0140741], thiazole synthase activity [GO:1990107]